{
  "term_label": "proteolysis",
  "gene_name": "Putative serine protease 42",
  "gene_symbol": "PRSS42P",
  "term_id": "GO:0006508",
  "gene": "UniProtKB:Q7Z5A4"
}